chaperone-mediated protein complex assembly [GO:0051131] (biological process) Regulation: regulated by regulation of chaperone-mediated protein complex assembly [GO:0090034]; positively regulated by positive regulation of chaperone-mediated protein complex assembly [GO:0090035] Definition: The aggregation, arrangement and bonding together of a set of components to form a protein complex, mediated by chaperone molecules that do not form part of the finished complex. Also known as: cellular chaperone-mediated protein complex assembly, protein complex assembly, multichaperone pathway, chaperone activity Relationships: is a type of protein-containing complex assembly [GO:0065003] Sources: GOC:ai